{
  "term_id": "GO:0071144",
  "gene": "UniProtKB:O15198",
  "gene_name": "Mothers against decapentaplegic homolog 9",
  "gene_symbol": "SMAD9",
  "term_label": "heteromeric SMAD protein complex"
}